pterin-4alpha-carbinolamine dehydratase activity [GO:0102434] (molecular function) References: PMID:18245455, PMID:20959559 Sources: GOC:pz Relationships: is a type of hydro-lyase activity [GO:0016836] Definition: Catalysis of the reaction: a 10-formyltetrahydrofolate-4a-carbinolamine = H2O + a 10-formyldihydrofolate.